{
  "term_label": "negative regulation of transcription by RNA polymerase II",
  "gene_name": "Melanoma-associated antigen B10",
  "term_id": "GO:0000122",
  "gene_symbol": "MAGEB10",
  "gene": "UniProtKB:Q96LZ2"
}